{
  "gene_symbol": "NME6",
  "term_id": "GO:0045839",
  "term_label": "negative regulation of mitotic nuclear division",
  "gene_name": "Nucleoside diphosphate kinase 6",
  "gene": "UniProtKB:O75414"
}